{
  "gene_symbol": "RECK",
  "gene": "UniProtKB:O95980",
  "gene_name": "Reversion-inducing cysteine-rich protein with Kazal motifs",
  "term_id": "GO:0002040",
  "term_label": "sprouting angiogenesis"
}